positive regulation of neuron remodeling [GO:1904801] (biological process) Definition: Any process that activates or increases the frequency, rate or extent of neuron remodeling. Also known as: positive regulation of neuron remodelling, positive regulation of neuronal remodeling, up regulation of neuron remodeling, up regulation of neuronal remodeling, up-regulation of neuron remodeling, up-regulation of neuronal remodeling, upregulation of neuron remodeling, upregulation of neuronal remodeling, activation of axon pruning, activation of neuron remodeling, activation of neuronal remodeling, positive regulation of axon pruning, up regulation of axon pruning, up-regulation of axon pruning, upregulation of axon pruning References: PMID:21609829 Sources: GOC:TermGenie, GO_REF:0000058 Relationships: is a type of GO:0014042; is a type of regulation of neuron remodeling [GO:1904799]; RO_0002213 neuron remodeling [GO:0016322] Note: cyy-1 in C. Elegans (P34624) in PMID:21609829 (inferred from mutant phenotype)